mycothiol metabolic process [GO:0010126] (biological process) Subtypes: mycothiol biosynthetic process [GO:0010125] Sources: GOC:pz Also known as: mycothiol metabolism Relationships: is_a sulfur compound metabolic process [GO:0006790]; is a type of GO:0016137 Definition: The chemical reactions and pathways involving mycothiol, which consists of N-acetyl-L-cysteine linked to a pseudodisaccharide, D-glucosamine and myo-inositol. Mycothiol is produced in actinomycetes like mycobacteria and serves similar functions to glutathione.